{
  "term_label": "endoplasmic reticulum",
  "gene": "UniProtKB:Q9UM00",
  "gene_name": "Calcium load-activated calcium channel",
  "gene_symbol": "TMCO1",
  "term_id": "GO:0005783"
}